Golgi calcium ion transmembrane transport [GO:0061856] (BP) Definition: A process in which a calcium ion is transported from one side of a Golgi membrane to the other by means of some agent such as a transporter or pore. References: PMID:21811607 Relationships: is a type of GO:0032472; is a type of calcium ion transmembrane transport [GO:0070588] Subtypes: release of sequestered calcium ion into cytosol by Golgi [GO:0061454]